{
  "term_label": "DNA-binding transcription factor activity, RNA polymerase II-specific",
  "gene": "UniProtKB:P51522",
  "gene_symbol": "ZNF83",
  "term_id": "GO:0000981",
  "gene_name": "Zinc finger protein 83"
}